{
  "gene_symbol": "KDELR2",
  "term_label": "endoplasmic reticulum",
  "term_id": "GO:0005783",
  "gene": "UniProtKB:P33947",
  "gene_name": "ER lumen protein-retaining receptor 2"
}